{
  "gene_symbol": "ZFP82",
  "gene": "UniProtKB:Q8N141",
  "gene_name": "Zinc finger protein 82 homolog",
  "term_id": "GO:0000978",
  "term_label": "RNA polymerase II cis-regulatory region sequence-specific DNA binding"
}